pulmonary myocardium development [GO:0003350] (biological process) Relationships: is_a striated muscle tissue development [GO:0014706]; is part of venous blood vessel development [GO:0060841] References: PMID:17638577 Sources: GOC:dph Definition: The progression of the pulmonary myocardium over time, from its initial formation to the mature structure. The pulmonary myocardium is the myocardial tissue present in the pulmonary vein.